NAD+-histone H2BE35 glutamate ADP-ribosyltransferase activity [GO:0140822] (molecular function) Definition: Catalysis of the transfer of ADP-ribose groups to the glutamate-35 residue of the N-terminal tail of histone H2B (or an equivalent residue). Relationships: is a type of NAD+-protein-glutamate ADP-ribosyltransferase activity [GO:0140807] References: PMID:32822587 Also known as: NAD+-histone H2B-E35 glutamate ADP-ribosyltransferase activity, NAD+-histone-glutamate ADP-ribosyltransferase activity (H2B-E35 specific) Note: Note that the residue position corresponds to the canonical human H2B histone (UniProtKB:P62807); this residue is conserved across all eukaryotes, but seems to be missing from Dictyostelium. Residue 1 is the first residue following removal of the initiating Methionine (Met). Note that each histone is encoded by multiple genes, and sequences may vary across different genes within an organism.